{
  "term_id": "GO:0048812",
  "gene_name": "Brain-derived neurotrophic factor",
  "gene_symbol": "BDNF",
  "term_label": "neuron projection morphogenesis",
  "gene": "UniProtKB:P23560"
}